{
  "term_label": "positive regulation of toll-like receptor 4 signaling pathway",
  "gene": "UniProtKB:Q8IWB7",
  "term_id": "GO:0034145",
  "gene_symbol": "WDFY1",
  "gene_name": "WD repeat and FYVE domain-containing protein 1"
}